{
  "gene_name": "Claudin-8",
  "gene_symbol": "CLDN8",
  "term_label": "paracellular tight junction channel activity",
  "gene": "UniProtKB:P56748",
  "term_id": "GO:0160187"
}